UDP-N-acetylmuramate-L-alanine ligase activity [GO:0008763] (molecular function) Definition: Catalysis of the reaction: L-alanine + ATP + UDP-N-acetylmuramate = ADP + 2 H+ + phosphate + UDP-N-acetylmuramoyl-L-alanine. Relationships: is a type of acid-amino acid ligase activity [GO:0016881] Sources: EC:6.3.2.8, RHEA:23372 Also known as: MurC synthetase activity, L-Ala ligase activity, L-alanine-adding enzyme activity, UDP-MurNAc:L-alanine ligase activity, UDP-N-acetylmuramate:L-alanine ligase (ADP-forming), UDP-N-acetylmuramoyl-L-alanine synthetase activity, UDP-N-acetylmuramoylalanine synthetase activity, UDP-N-acetylmuramyl:L-alanine ligase activity, UDP-acetylmuramyl-L-alanine synthetase activity, UDPMurNAc-L-alanine synthetase activity, alanine-adding enzyme activity, uridine 5'-diphosphate-N-acetylmuramyl-L-alanine synthetase activity, uridine diphosphate N-acetylmuramate:L-alanine ligase activity, uridine diphospho-N-acetylmuramoylalanine synthetase activity, uridine-diphosphate-N-acetylmuramate:L-alanine ligase activity